sperm head [GO:0061827] (cellular component) References: PMID:22797892, PMID:24665388 Definition: The part of the late spermatid or spermatozoon that contains the nucleus and acrosome. Relationships: is a type of cellular anatomical structure [GO:0110165]